{
  "gene_name": "Interleukin-8",
  "term_id": "GO:0030593",
  "term_label": "neutrophil chemotaxis",
  "gene_symbol": "CXCL8",
  "gene": "UniProtKB:P10145"
}